{
  "gene_symbol": "MT1H",
  "term_id": "GO:0010273",
  "gene": "UniProtKB:P80294",
  "term_label": "detoxification of copper ion",
  "gene_name": "Metallothionein-1H"
}